negative regulation of penile erection [GO:0060407] (biological process) Definition: Any process that stops, prevents, or reduces the rate, frequency or extent of penile erection. Penile erection is the hardening, enlarging and rising of the penis which often occurs in the sexually aroused male and enables sexual intercourse. Achieved by increased inflow of blood into the vessels of erectile tissue, and decreased outflow. Sources: GOC:dph, GOC:tb Relationships: is a type of negative regulation of multicellular organismal process [GO:0051241]; is a type of regulation of penile erection [GO:0060405]; is a type of negative regulation of reproductive process [GO:2000242]; negatively regulates GO:0043084